{
  "gene": "UniProtKB:P32019",
  "term_label": "phosphatidylinositol-4,5-bisphosphate 5-phosphatase activity",
  "term_id": "GO:0004439",
  "gene_name": "Type II inositol 1,4,5-trisphosphate 5-phosphatase",
  "gene_symbol": "INPP5B"
}